{
  "gene_name": "Adenomatous polyposis coli protein 2",
  "gene_symbol": "APC2",
  "gene": "UniProtKB:O95996",
  "term_label": "microtubule binding",
  "term_id": "GO:0008017"
}